{
  "gene_name": "Keratin, type I cytoskeletal 20",
  "gene": "UniProtKB:P35900",
  "term_id": "GO:0030280",
  "term_label": "structural constituent of skin epidermis",
  "gene_symbol": "KRT20"
}